{
  "term_label": "DNA-binding transcription factor activity, RNA polymerase II-specific",
  "term_id": "GO:0000981",
  "gene": "UniProtKB:Q7Z398",
  "gene_symbol": "ZNF550",
  "gene_name": "Zinc finger protein 550"
}